{
  "term_id": "GO:0055085",
  "gene_name": "Sodium-dependent lysophosphatidylcholine symporter 1",
  "gene_symbol": "MFSD2A",
  "term_label": "transmembrane transport",
  "gene": "UniProtKB:Q8NA29"
}